structural constituent of muscle [GO:0008307] (MF) Definition: The action of a molecule that contributes to the structural integrity of a muscle fiber. Relationships: is a type of GO:0005198 Sources: GOC:mah